ATPase-coupled antimonite transmembrane transporter activity [GO:0042961] (molecular function) Definition: Enables the transfer of a solute or solutes from one side of a membrane to the other according to the reaction: ATP + H2O + antimonite(in) = ADP + phosphate + antimonite(out). Relationships: is a type of antimonite transmembrane transporter activity [GO:0015104]; is a type of ATPase-coupled transmembrane transporter activity [GO:0042626] Sources: EC:7.3.2.7 Also known as: ATP-dependent antimonite transporter activity, antimonite-transporting ATPase activity